positive regulation of nonadec-1-ene biosynthetic process [GO:1900937] (biological process) Also known as: activation of nonadec-1-ene anabolism, activation of nonadec-1-ene biosynthesis, activation of nonadec-1-ene formation, activation of nonadec-1-ene synthesis, positive regulation of nonadec-1-ene anabolism, positive regulation of nonadec-1-ene biosynthesis, positive regulation of nonadec-1-ene formation, positive regulation of nonadec-1-ene synthesis, up regulation of nonadec-1-ene anabolism, up regulation of nonadec-1-ene biosynthesis, up regulation of nonadec-1-ene biosynthetic process, up regulation of nonadec-1-ene formation, up regulation of nonadec-1-ene synthesis, up-regulation of nonadec-1-ene anabolism, up-regulation of nonadec-1-ene biosynthesis, up-regulation of nonadec-1-ene biosynthetic process, up-regulation of nonadec-1-ene formation, up-regulation of nonadec-1-ene synthesis, upregulation of nonadec-1-ene anabolism, upregulation of nonadec-1-ene biosynthesis, upregulation of nonadec-1-ene biosynthetic process, upregulation of nonadec-1-ene formation, upregulation of nonadec-1-ene synthesis, activation of nonadec-1-ene biosynthetic process Definition: Any process that activates or increases the frequency, rate or extent of nonadec-1-ene biosynthetic process. Relationships: is a type of GO:1900913; is a type of regulation of nonadec-1-ene biosynthetic process [GO:1900935]; RO_0002213 nonadec-1-ene biosynthetic process [GO:1900877] Sources: GOC:TermGenie, GOC:mengo_curators